regulation of high-density lipoprotein particle clearance [GO:0010982] (biological process) Definition: Any process that modulates the rate, frequency or extent of high-density lipoprotein particle clearance. High-density lipoprotein particle clearance is the process in which a high-density lipoprotein particle is removed from the blood via receptor-mediated endocytosis and its constituent parts degraded. Sources: GOC:BHF, GOC:dph, GOC:tb Subtypes: GO:0010983, negative regulation of high-density lipoprotein particle clearance [GO:0010987] Relationships: is a type of regulation of lipoprotein particle clearance [GO:0010984]; regulates high-density lipoprotein particle clearance [GO:0034384]